{
  "gene_symbol": "FOXR1",
  "gene_name": "Forkhead box protein R1",
  "term_id": "GO:1990837",
  "term_label": "sequence-specific double-stranded DNA binding",
  "gene": "UniProtKB:Q6PIV2"
}